{
  "gene_symbol": "ZEB1",
  "term_id": "GO:0007417",
  "gene": "UniProtKB:P37275",
  "term_label": "central nervous system development",
  "gene_name": "Zinc finger E-box-binding homeobox 1"
}